{
  "gene_name": "Prostaglandin E2 receptor EP2 subtype",
  "gene": "UniProtKB:P43116",
  "gene_symbol": "PTGER2",
  "term_id": "GO:0007204",
  "term_label": "positive regulation of cytosolic calcium ion concentration"
}